fibroblast growth factor binding [GO:0017134] (molecular function) References: PMID:9806903 Relationships: is a type of GO:0019838 Also known as: FGF binding, FGF 1 binding, FGF 2 binding, FGF 3 binding, FGF 4 binding, FGF 5 binding, FGF 6 binding, fibroblast growth factor 1 binding, fibroblast growth factor 2 binding, fibroblast growth factor 3 binding, fibroblast growth factor 4 binding, fibroblast growth factor 5 binding, fibroblast growth factor 6 binding Definition: Binding to a fibroblast growth factor.